{
  "term_id": "GO:0007179",
  "term_label": "transforming growth factor beta receptor signaling pathway",
  "gene_symbol": "TGFBR1",
  "gene": "UniProtKB:P36897",
  "gene_name": "TGF-beta receptor type-1"
}